{
  "gene_name": "Macrosialin",
  "gene_symbol": "CD68",
  "gene": "UniProtKB:P34810",
  "term_id": "GO:0031902",
  "term_label": "late endosome membrane"
}